positive regulation of transcription from a mobile element promoter [GO:0061435] (biological process) Relationships: is a type of GO:0045893 Definition: Any process that activates or increases the frequency, rate or extent of transcription from a mobile element promoter. References: PMID:12230120, PMID:9271107 Sources: GOC:dph